zerumbone synthase activity [GO:0102069] (molecular function) Relationships: is_a oxidoreductase activity, acting on the CH-OH group of donors, NAD or NADP as acceptor [GO:0016616] Definition: Catalysis of the reaction: 8-hydroxy-alpha-humulene + NAD = zerumbone + NADH + H+. Sources: EC:1.1.1.326, GOC:pz